{
  "gene_symbol": "KLK6",
  "term_label": "extracellular space",
  "term_id": "GO:0005615",
  "gene_name": "Kallikrein-6",
  "gene": "UniProtKB:Q92876"
}